{
  "gene_symbol": "TH",
  "term_id": "GO:0006585",
  "gene_name": "Tyrosine 3-monooxygenase",
  "term_label": "dopamine biosynthetic process from tyrosine",
  "gene": "UniProtKB:P07101"
}